{
  "term_label": "endoplasmic reticulum to Golgi vesicle-mediated transport",
  "term_id": "GO:0006888",
  "gene": "UniProtKB:Q9Y282",
  "gene_symbol": "ERGIC3",
  "gene_name": "Endoplasmic reticulum-Golgi intermediate compartment protein 3"
}